{
  "gene": "UniProtKB:Q8IYA8",
  "term_id": "GO:0042138",
  "term_label": "meiotic DNA double-strand break formation",
  "gene_name": "Interactor of HORMAD1 protein 1",
  "gene_symbol": "IHO1"
}